{
  "gene_name": "E3 ubiquitin-protein ligase RNF149",
  "term_label": "late endosome",
  "term_id": "GO:0005770",
  "gene_symbol": "RNF149",
  "gene": "UniProtKB:Q8NC42"
}